connective tissue growth factor production [GO:0032601] (biological process) Relationships: is a type of cytokine production [GO:0001816] Regulation: RO_0002211 by regulation of connective tissue growth factor production [GO:0032643]; negatively regulated by negative regulation of connective tissue growth factor production [GO:0032683]; positively regulated by positive regulation of connective tissue growth factor production [GO:0032723] Sources: GOC:mah Definition: The appearance of connective tissue growth factor due to biosynthesis or secretion following a cellular stimulus, resulting in an increase in its intracellular or extracellular levels. Also known as: CCN2 production, CTGF production, Fisp12 production, Hcs24 production, IGFBP8 production, hypertrophic chondrocyte-specific gene product 24 production